{
  "gene_symbol": "POLRMT",
  "gene_name": "DNA-directed RNA polymerase, mitochondrial",
  "term_id": "GO:0003899",
  "gene": "UniProtKB:O00411",
  "term_label": "DNA-directed RNA polymerase activity"
}